{
  "gene_name": "Protein cornichon homolog 3",
  "gene_symbol": "CNIH3",
  "term_label": "synapse",
  "term_id": "GO:0045202",
  "gene": "UniProtKB:Q8TBE1"
}